response to monoamine [GO:0071867] (biological process) Sources: GOC:mah Subtypes: response to iloperidone [GO:0036287], cellular response to monoamine stimulus [GO:0071868], GO:0071869, GO:1904014 Relationships: is a type of response to nitrogen compound [GO:1901698] Also known as: response to monoamine stimulus Definition: Any process that results in a change in state or activity of a cell or an organism (in terms of movement, secretion, enzyme production, gene expression, etc.) as a result of a monoamine stimulus. A monoamine is any of a group of molecular messengers that contain one amino group that is connected to an aromatic ring by ethylene group (-CH2-CH2-). Monoamines are derived from the aromatic amino acids phenylalanine, tyrosine, histidine and tryptophan.